leukocyte tethering or rolling [GO:0050901] (biological process) Regulation: RO_0002211 by regulation of leukocyte tethering or rolling [GO:1903236]; negatively regulated by negative regulation of leukocyte tethering or rolling [GO:1903237]; positively regulated by positive regulation of leukocyte tethering or rolling [GO:1903238] Relationships: is a type of GO:0061756; is part of GO:0045123 References: PMID:14680625, PMID:14708592, PMID:7507411, PMID:8600538 Sources: GOC:bf, ISBN:0781735149, Wikipedia:Leukocyte_extravasation Definition: Transient adhesive interactions between leukocytes and endothelial cells lining blood vessels. Carbohydrates on circulating leukocytes bind selectins on the vessel wall causing the leukocytes to slow down and roll along the inner surface of the vessel wall. During this rolling motion, transitory bonds are formed and broken between selectins and their ligands. Typically the first step in cellular extravasation (the movement of leukocytes out of the circulatory system, towards the site of tissue damage or infection).